{
  "gene_symbol": "GUK1",
  "term_id": "GO:0004385",
  "term_label": "GMP kinase activity",
  "gene_name": "Guanylate kinase",
  "gene": "UniProtKB:Q16774"
}